{
  "gene_symbol": "SNAP91",
  "gene": "UniProtKB:O60641",
  "gene_name": "Clathrin coat assembly protein AP180",
  "term_id": "GO:0000149",
  "term_label": "SNARE binding"
}